protein-lysine 6-oxidase activity [GO:0004720] (molecular function) Sources: EC:1.4.3.13 Relationships: is a type of diamine oxidase activity [GO:0052597]; is a type of GO:0140096 Definition: Catalysis of the reaction: peptidyl-L-lysyl-peptide + H2O + O2 = peptidyl-allysyl-peptide + NH3 + hydrogen peroxide. Also known as: lysyl oxidase activity, protein-L-lysine:oxygen 6-oxidoreductase (deaminating)